neuromuscular junction development [GO:0007528] (biological process) Regulation: regulated by regulation of neuromuscular junction development [GO:1904396]; negatively regulated by GO:1904397; positively regulated by positive regulation of neuromuscular junction development [GO:1904398] Definition: A process that is carried out at the cellular level which results in the assembly, arrangement of constituent parts, or disassembly of a neuromuscular junction. Sources: GOC:mtg_OBO2OWL_2013 Also known as: neuromuscular junction organization, NMJ stability, neuromuscular junction stability Subtypes: GO:0051124, GO:0098529 Relationships: is a type of synapse organization [GO:0050808]